{
  "gene_symbol": "TLCD2",
  "term_label": "phospholipid homeostasis",
  "gene_name": "TLC domain-containing protein 2",
  "term_id": "GO:0055091",
  "gene": "UniProtKB:A6NGC4"
}